galactolipid metabolic process [GO:0019374] (biological process) Definition: The chemical reactions and pathways involving galactolipids, any glycolipid containing one of more residues of galactose and/or N-acetylgalactosamine. Sources: ISBN:0198506732 Relationships: is a type of glycolipid metabolic process [GO:0006664] Also known as: galactolipid metabolism Subtypes: galactosylceramide metabolic process [GO:0006681], galactolipid biosynthetic process [GO:0019375], galactolipid catabolic process [GO:0019376]